{
  "gene_symbol": "MED23",
  "gene": "UniProtKB:Q9ULK4",
  "gene_name": "Mediator of RNA polymerase II transcription subunit 23",
  "term_id": "GO:0016592",
  "term_label": "mediator complex"
}